negative regulation of cellular response to macrophage colony-stimulating factor stimulus [GO:1903973] (biological process) References: PMID:19100238 Sources: GOC:BHF, GOC:TermGenie, GOC:nc, GO_REF:0000058 Relationships: is a type of negative regulation of response to macrophage colony-stimulating factor [GO:1903970]; is a type of regulation of cellular response to macrophage colony-stimulating factor stimulus [GO:1903972]; negatively regulates cellular response to macrophage colony-stimulating factor stimulus [GO:0036006] Definition: Any process that stops, prevents or reduces the frequency, rate or extent of cellular response to macrophage colony-stimulating factor stimulus. Also known as: down regulation of cellular response to M-CSF stimulus, down regulation of cellular response to macrophage colony-stimulating factor, down regulation of cellular response to macrophage colony-stimulating factor stimulus, down-regulation of cellular response to M-CSF stimulus, down-regulation of cellular response to macrophage colony-stimulating factor, down-regulation of cellular response to macrophage colony-stimulating factor stimulus, downregulation of cellular response to M-CSF stimulus, downregulation of cellular response to macrophage colony-stimulating factor, downregulation of cellular response to macrophage colony-stimulating factor stimulus, negative regulation of cellular response to M-CSF stimulus, negative regulation of cellular response to macrophage colony-stimulating factor, inhibition of cellular response to M-CSF stimulus, inhibition of cellular response to macrophage colony-stimulating factor, inhibition of cellular response to macrophage colony-stimulating factor stimulus